{
  "gene_symbol": "NTN3",
  "term_label": "DNA-binding transcription factor activity, RNA polymerase II-specific",
  "gene_name": "Netrin-3",
  "gene": "UniProtKB:O00634",
  "term_id": "GO:0000981"
}